{
  "gene_name": "26S proteasome non-ATPase regulatory subunit 13",
  "term_id": "GO:0005198",
  "gene": "UniProtKB:Q9UNM6",
  "term_label": "structural molecule activity",
  "gene_symbol": "PSMD13"
}